{
  "gene_symbol": "SETD7",
  "gene_name": "Histone-lysine N-methyltransferase SETD7",
  "gene": "UniProtKB:Q8WTS6",
  "term_label": "nucleus",
  "term_id": "GO:0005634"
}